{
  "gene_name": "Dr1-associated corepressor",
  "term_id": "GO:0016251",
  "gene_symbol": "DRAP1",
  "gene": "UniProtKB:Q14919",
  "term_label": "RNA polymerase II general transcription initiation factor activity"
}